{
  "gene_symbol": "ERP29",
  "term_id": "UNKNOWN:0001",
  "gene": "UniProtKB:P30040",
  "term_label": "Unknown molecular function",
  "gene_name": "Endoplasmic reticulum resident protein 29"
}